{
  "term_label": "nucleus",
  "gene": "UniProtKB:Q9H5J0",
  "gene_name": "Zinc finger and BTB domain-containing protein 3",
  "term_id": "GO:0005634",
  "gene_symbol": "ZBTB3"
}